{
  "term_label": "histone binding",
  "gene_name": "SWI_SNF complex subunit SMARCC2",
  "term_id": "GO:0042393",
  "gene": "UniProtKB:Q8TAQ2",
  "gene_symbol": "SMARCC2"
}